{
  "gene_symbol": "CRHR1",
  "term_id": "GO:0015056",
  "term_label": "corticotrophin-releasing factor receptor activity",
  "gene_name": "Corticotropin-releasing factor receptor 1",
  "gene": "UniProtKB:P34998"
}